{
  "gene_name": "Protein Niban 3",
  "gene": "UniProtKB:Q86XR2",
  "term_label": "Unknown molecular function",
  "gene_symbol": "NIBAN3",
  "term_id": "UNKNOWN:0001"
}